response to chromate [GO:0046687] (biological process) Also known as: chromate sensitivity/resistance Definition: Any process that results in a change in state or activity of a cell or an organism (in terms of movement, secretion, enzyme production, gene expression, etc.) as a result of a chromate stimulus. Subtypes: cellular response to chromate [GO:0071247] Relationships: is a type of response to oxygen-containing compound [GO:1901700] Sources: ISBN:0721662544